{
  "gene_symbol": "CEP295",
  "gene": "UniProtKB:Q9C0D2",
  "gene_name": "Centrosomal protein of 295 kDa",
  "term_label": "Unknown molecular function",
  "term_id": "UNKNOWN:0001"
}